{
  "gene_symbol": "PSMC3IP",
  "term_id": "GO:0003690",
  "gene_name": "Homologous-pairing protein 2 homolog",
  "gene": "UniProtKB:Q9P2W1",
  "term_label": "double-stranded DNA binding"
}